negative regulation of insulin secretion involved in cellular response to glucose stimulus [GO:0061179] (biological process) Also known as: negative regulation of insulin secretion involved in cellular response to glucose, negative regulation of insulin secretion in response to glucose Definition: Any process that decreases the frequency, rate or extent of the regulated release of insulin that contributes to the response of a cell to glucose. Sources: GOC:BHF, GOC:dph Relationships: is a type of negative regulation of insulin secretion [GO:0046676]; is a type of negative regulation of response to stimulus [GO:0048585]; is a type of regulation of insulin secretion involved in cellular response to glucose stimulus [GO:0061178]; negatively regulates insulin secretion involved in cellular response to glucose stimulus [GO:0035773]